cyanophycin synthetase activity (L-aspartate-adding) [GO:0071160] (molecular function) Relationships: is_a cyanophycin synthetase activity [GO:0043860] Sources: EC:6.3.2.29 Definition: Catalysis of the reaction: ATP + [L-Asp(4-L-Arg)]n + L-Asp = ADP + phosphate + [L-Asp(4-L-Arg)]n-L-Asp.